{
  "gene_name": "Phosphatidylcholine-sterol acyltransferase",
  "gene": "UniProtKB:P04180",
  "term_id": "GO:0005615",
  "gene_symbol": "LCAT",
  "term_label": "extracellular space"
}